{
  "gene": "UniProtKB:Q13705",
  "term_label": "pattern specification process",
  "term_id": "GO:0007389",
  "gene_name": "Activin receptor type-2B",
  "gene_symbol": "ACVR2B"
}